6-hydroxynicotinate reductase activity [GO:0047595] (molecular function) Also known as: 1,4,5,6-tetrahydro-6-oxonicotinate:ferredoxin oxidoreductase activity, 6-hydroxynicotinic reductase activity, 6-oxo-1,4,5,6-tetrahydronicotinate:ferredoxin oxidoreductase activity, 6-oxotetrahydro-nicotinate dehydrogenase activity, 6-oxotetrahydronicotinate dehydrogenase activity, HNA reductase activity Sources: EC:1.3.7.1, MetaCyc:6-HYDROXYNICOTINATE-REDUCTASE-RXN Definition: Catalysis of the reaction: 1,4,5,6-tetrahydro-6-oxonicotinate + oxidized ferredoxin = 6-hydroxynicotinate + reduced ferredoxin. Relationships: is a type of oxidoreductase activity, acting on the CH-CH group of donors, iron-sulfur protein as acceptor [GO:0016636]